{
  "gene_symbol": "ADAP2",
  "term_id": "GO:0005886",
  "gene": "UniProtKB:Q9NPF8",
  "term_label": "plasma membrane",
  "gene_name": "Arf-GAP with dual PH domain-containing protein 2"
}